{
  "gene": "UniProtKB:Q8N0X4",
  "gene_name": "Citramalyl-CoA lyase, mitochondrial",
  "gene_symbol": "CLYBL",
  "term_id": "GO:0047777",
  "term_label": "(S)-citramalyl-CoA lyase activity"
}